{
  "gene_name": "Platelet-derived growth factor subunit A",
  "gene_symbol": "PDGFA",
  "gene": "UniProtKB:P04085",
  "term_label": "positive regulation of ERK1 and ERK2 cascade",
  "term_id": "GO:0070374"
}